{
  "term_label": "NatB complex",
  "gene": "UniProtKB:Q14CX7",
  "gene_name": "N-alpha-acetyltransferase 25, NatB auxiliary subunit",
  "gene_symbol": "NAA25",
  "term_id": "GO:0031416"
}